{
  "gene_symbol": "RPS24",
  "gene": "UniProtKB:P62847",
  "term_label": "cytoplasmic translation",
  "gene_name": "Small ribosomal subunit protein eS24",
  "term_id": "GO:0002181"
}